meiosis I nuclear membrane reassembly [GO:0051334] (biological process) Also known as: meiosis I nuclear envelope reassembly Relationships: is a type of GO:0051333; is part of meiosis I [GO:0007127] Sources: GOC:ai Definition: The reformation of the nuclear membranes during meiosis I.